{
  "term_id": "GO:0008191",
  "gene_symbol": "SPOCK1",
  "gene_name": "Testican-1",
  "gene": "UniProtKB:Q08629",
  "term_label": "metalloendopeptidase inhibitor activity"
}